negative regulation of hydrogen peroxide catabolic process [GO:2000296] (biological process) Sources: GOC:BHF Relationships: is a type of negative regulation of catabolic process [GO:0009895]; is a type of negative regulation of hydrogen peroxide metabolic process [GO:0010727]; is a type of regulation of hydrogen peroxide catabolic process [GO:2000295]; negatively regulates hydrogen peroxide catabolic process [GO:0042744] Definition: Any process that stops, prevents or reduces the frequency, rate or extent of hydrogen peroxide catabolic process. Also known as: negative regulation of H2O2 catabolic process, negative regulation of hydrogen peroxide breakdown, negative regulation of hydrogen peroxide catabolism, negative regulation of hydrogen peroxide degradation, negative regulation of H2O2 scavenging, negative regulation of detoxification of H2O2, negative regulation of detoxification of hydrogen peroxide, negative regulation of hydrogen peroxide removal, negative regulation of hydrogen peroxide scavenging